{
  "gene": "UniProtKB:Q8NGQ5",
  "gene_symbol": "OR9Q1",
  "term_label": "G protein-coupled receptor signaling pathway",
  "gene_name": "Olfactory receptor 9Q1",
  "term_id": "GO:0007186"
}